organelle localization by membrane tethering [GO:0140056] (biological process) Definition: The process by which an organelle membrane interacts with another membrane via molecular tethers that physically bridge the two membranes and attach them to each other. Subtypes: peroxisome-chloroplast membrane tethering [GO:0010381], autophagosome membrane docking [GO:0016240], vesicle docking [GO:0048278], endoplasmic reticulum-plasma membrane tethering [GO:0061817], endoplasmic reticulum-peroxisome tethering [GO:0062095], nucleus-vacuole junction assembly [GO:0071562], ciliary basal body-plasma membrane docking [GO:0097711], vacuole-mitochondria membrane tethering [GO:0140057], mitochondrion-endoplasmic reticulum membrane tethering [GO:1990456], vacuole-ER tethering [GO:1990854] Relationships: is a type of membrane docking [GO:0022406]; is a type of organelle localization [GO:0051640] References: PMID:27875684